{
  "gene_symbol": "SLC35D3",
  "term_label": "transmembrane transport",
  "term_id": "GO:0055085",
  "gene_name": "Solute carrier family 35 member D3",
  "gene": "UniProtKB:Q5M8T2"
}